{
  "gene_symbol": "PAGR1",
  "term_label": "MLL3/4 complex",
  "term_id": "GO:0044666",
  "gene_name": "PAXIP1-associated glutamate-rich protein 1",
  "gene": "UniProtKB:Q9BTK6"
}